{
  "gene": "UniProtKB:Q86SH4",
  "gene_symbol": "PRNT",
  "term_label": "Unknown molecular function",
  "gene_name": "Putative testis-specific prion protein",
  "term_id": "UNKNOWN:0001"
}